{
  "gene_name": "T cell receptor beta joining 2-5",
  "term_label": "Unknown molecular function",
  "gene_symbol": "TRBJ2-5",
  "gene": "UniProtKB:A0A0A0MTA4",
  "term_id": "UNKNOWN:0001"
}